endoplasmic reticulum-vacuole membrane contact site [GO:0098853] (cellular component) Relationships: is_a organelle membrane contact site [GO:0044232] References: PMID:26283797 Sources: GOC:dos Definition: A zone of apposition between endoplasmic-reticulum and lytic vacuole membranes, structured by bridging complexes. Also known as: ER-vacuole membrane contact site